{
  "gene": "UniProtKB:Q96RT7",
  "term_label": "spindle assembly",
  "gene_name": "Gamma-tubulin complex component 6",
  "term_id": "GO:0051225",
  "gene_symbol": "TUBGCP6"
}